{
  "term_label": "actin filament-based movement",
  "gene_symbol": "MYO6",
  "gene_name": "Unconventional myosin-VI",
  "gene": "UniProtKB:Q9UM54",
  "term_id": "GO:0030048"
}